{
  "gene_symbol": "FCRL4",
  "gene": "UniProtKB:Q96PJ5",
  "gene_name": "Fc receptor-like protein 4",
  "term_label": "external side of plasma membrane",
  "term_id": "GO:0009897"
}